{
  "gene_symbol": "ZNF549",
  "term_id": "GO:0006357",
  "gene": "UniProtKB:Q6P9A3",
  "term_label": "regulation of transcription by RNA polymerase II",
  "gene_name": "Zinc finger protein 549"
}